{
  "term_id": "GO:0031012",
  "term_label": "extracellular matrix",
  "gene": "UniProtKB:Q9UKU9",
  "gene_name": "Angiopoietin-related protein 2",
  "gene_symbol": "ANGPTL2"
}